regulation of female receptivity [GO:0045924] (biological process) Definition: Any process that modulates the frequency, rate or extent of the willingness or readiness of a female to receive male advances. Sources: GOC:dph, GOC:go_curators, GOC:tb Relationships: is a type of female mating behavior [GO:0060180]; is a type of regulation of biological quality [GO:0065008] Also known as: female receptivity Subtypes: negative regulation of female receptivity [GO:0007621], positive regulation of female receptivity [GO:0045925], GO:0046008